{
  "term_id": "UNKNOWN:0001",
  "gene_name": "Cysteine-rich secretory protein 2",
  "gene_symbol": "CRISP2",
  "term_label": "Unknown molecular function",
  "gene": "UniProtKB:P16562"
}